uridine:proton symporter activity [GO:0015394] (molecular function) Relationships: is a type of GO:0015213; is a type of nucleoside:proton symporter activity [GO:0015506] Definition: Enables the transfer of a solute or solutes from one side of a membrane to the other according to the reaction: uridine(out) + H+(out) = uridine(in) + H+(in). Sources: GOC:mtg_transport Also known as: uridine:hydrogen ion symporter activity, nucleoside (uridine) permease activity